{
  "gene": "UniProtKB:P35908",
  "gene_symbol": "KRT2",
  "term_id": "GO:0045095",
  "gene_name": "Keratin, type II cytoskeletal 2 epidermal",
  "term_label": "keratin filament"
}